{
  "gene": "UniProtKB:O95047",
  "gene_symbol": "OR2A4",
  "term_label": "odorant binding",
  "gene_name": "Olfactory receptor 2A4",
  "term_id": "GO:0005549"
}